{
  "gene": "UniProtKB:Q96LA5",
  "term_label": "cell surface receptor signaling pathway",
  "gene_symbol": "FCRL2",
  "term_id": "GO:0007166",
  "gene_name": "Fc receptor-like protein 2"
}